anatomical structure morphogenesis [GO:0009653] (biological process) Relationships: is a type of developmental process [GO:0032502]; is part of anatomical structure development [GO:0048856] Sources: GOC:go_curators, ISBN:0521436125 Also known as: embryogenesis and morphogenesis, anatomical structure organization, morphogenesis Subtypes: GO:0000902, morphogenesis of a branching structure [GO:0001763], lymphangiogenesis [GO:0001946], GO:0002089, GO:0003142, membranous septum morphogenesis [GO:0003149], outflow tract morphogenesis [GO:0003151], endocardium morphogenesis [GO:0003160], heart valve morphogenesis [GO:0003179], cardiac chamber morphogenesis [GO:0003206], heart wedging [GO:0003297], establishment of tissue polarity [GO:0007164], GO:0007440, hindgut morphogenesis [GO:0007442], GO:0009886, animal organ morphogenesis [GO:0009887], shoot system morphogenesis [GO:0010016], body morphogenesis [GO:0010171], central nervous system morphogenesis [GO:0021551], hindbrain morphogenesis [GO:0021575], medulla oblongata morphogenesis [GO:0021579], GO:0021583, cerebellum morphogenesis [GO:0021587], rhombomere morphogenesis [GO:0021593], GO:0021602, cerebellar granular layer morphogenesis [GO:0021683], cerebellar molecular layer morphogenesis [GO:0021687], cerebellar Purkinje cell layer morphogenesis [GO:0021692], cerebellar cortex morphogenesis [GO:0021696], locus ceruleus morphogenesis [GO:0021704], inferior olivary nucleus morphogenesis [GO:0021714], superior olivary nucleus morphogenesis [GO:0021719], GO:0031069, GO:0031288, appendage morphogenesis [GO:0035107], tube morphogenesis [GO:0035239], GO:0035277, dorsal motor nucleus of vagus nerve morphogenesis [GO:0035762], ascending aorta morphogenesis [GO:0035910], GO:0035911, foramen ovale closure [GO:0035922], GO:0036022, lymph vessel morphogenesis [GO:0036303], GO:0036304, post-anal tail morphogenesis [GO:0036342], sorocarp stalk morphogenesis [GO:0036360], embryonic morphogenesis [GO:0048598], GO:0048729, compound eye corneal lens morphogenesis [GO:0048750], swim bladder inflation [GO:0048798], diencephalon morphogenesis [GO:0048852], forebrain morphogenesis [GO:0048853], adenohypophysis morphogenesis [GO:0048855], cell projection morphogenesis [GO:0048858], retina morphogenesis in camera-type eye [GO:0060042], head morphogenesis [GO:0060323], face morphogenesis [GO:0060325], cardiac septum morphogenesis [GO:0060411], GO:0060463, nipple morphogenesis [GO:0060658], prostate gland stromal morphogenesis [GO:0060741], leaflet morphogenesis [GO:0060794], iris morphogenesis [GO:0061072], ciliary body morphogenesis [GO:0061073], fungiform papilla morphogenesis [GO:0061197], retina vasculature morphogenesis in camera-type eye [GO:0061299], cerebellum vasculature morphogenesis [GO:0061301], trabecula morphogenesis [GO:0061383], renal system vasculature morphogenesis [GO:0061438], kidney vasculature morphogenesis [GO:0061439], ectodermal placode morphogenesis [GO:0071697], GO:0071729, nephron morphogenesis [GO:0072028], comma-shaped body morphogenesis [GO:0072049], GO:0072050, glomerulus morphogenesis [GO:0072102], male anatomical structure morphogenesis [GO:0090598], plant epidermis morphogenesis [GO:0090626], post-embryonic plant morphogenesis [GO:0090698], craniofacial suture morphogenesis [GO:0097094], GO:0140509, midbrain morphogenesis [GO:1904693], atrioventricular canal morphogenesis [GO:1905222], epicardium morphogenesis [GO:1905223], plant organ morphogenesis [GO:1905392], hard palate morphogenesis [GO:1905748], nematode pharyngeal gland morphogenesis [GO:1905905], GO:1990522 Definition: The process in which anatomical structures are generated and organized. Morphogenesis pertains to the creation of form. Regulation: regulated by regulation of anatomical structure morphogenesis [GO:0022603]